karyomere [GO:0061468] (cellular component) Definition: A membrane-bound intermediate cleavage-stage structure of individual or groups of chromosomes that coalesces and fuses with other karyomeres to form a nucleus during interphase. Karyomere formation occurs in blastomeres undergoing rapid cell division. References: PMID:12734396, PMID:22863006 Sources: GOC:dph Relationships: is a type of intracellular membrane-bounded organelle [GO:0043231]